{
  "term_label": "ubiquitin protein ligase activity",
  "gene_symbol": "ZNRF3",
  "gene": "UniProtKB:Q9ULT6",
  "gene_name": "E3 ubiquitin-protein ligase ZNRF3",
  "term_id": "GO:0061630"
}